{
  "gene_name": "RNA binding protein fox-1 homolog 1",
  "gene": "UniProtKB:Q9NWB1",
  "term_id": "GO:0005737",
  "term_label": "cytoplasm",
  "gene_symbol": "RBFOX1"
}